Schwann cell development [GO:0014044] (biological process) Definition: The process aimed at the progression of a Schwann cell over time, from initial commitment of the cell to a specific fate, to the fully functional differentiated cell. Schwann cells are found in the peripheral nervous system, where they insulate neurons and axons, and regulate the environment in which neurons function. Sources: GOC:dgh, GOC:ef Relationships: is a type of glial cell development [GO:0021782]; is part of Schwann cell differentiation [GO:0014037]